glutathione transmembrane transport [GO:0034775] (biological process) Definition: A process in which glutathione is transported across a membrane. Relationships: is a type of glutathione transport [GO:0034635]; is a type of GO:0035443 Also known as: glutathione membrane transport, transmembrane glutathione transport Subtypes: glutathione transmembrane import into vacuole [GO:0071996], GO:0098709, glutathione import into mitochondrion [GO:0160007] Sources: GOC:mah Note: Note that this term is not intended for use in annotating lateral movement within membranes.